{
  "gene": "UniProtKB:A0A578",
  "gene_name": "T cell receptor beta variable 5-1",
  "gene_symbol": "TRBV5-1",
  "term_label": "cell surface receptor signaling pathway",
  "term_id": "GO:0007166"
}